{
  "gene_symbol": "OASL",
  "term_label": "cytosol",
  "term_id": "GO:0005829",
  "gene_name": "2'-5'-oligoadenylate synthase-like protein",
  "gene": "UniProtKB:Q15646"
}